dihydroxyfumarate decarboxylase activity [GO:0047858] (molecular function) Relationships: is a type of carboxy-lyase activity [GO:0016831] Also known as: dihydroxyfumarate carboxy-lyase (tartronate-semialdehyde-forming), dihydroxyfumarate carboxy-lyase activity Sources: EC:4.1.1.54, RHEA:13845 Definition: Catalysis of the reaction: dihydroxyfumarate + H+ = 2-hydroxy-3-oxopropanoate + CO2.